anterograde axonal transport of mitochondrion [GO:0098957] (biological process) Sources: GOC:dos Also known as: anterograde axon transport of mitochondria Relationships: is a type of GO:0008089; is a type of axonal transport of mitochondrion [GO:0019896] Regulation: regulated by GO:0061880; positively regulated by positive regulation of anterograde axonal transport of mitochondrion [GO:0061881]; RO_0002212 by GO:0061882 Definition: The directed movement of mitochondria along microtubules in axons away from the cell body and towards the presynapse.